extrinsic component of presynaptic membrane [GO:0098888] (cellular component) Definition: The component of the presynaptic membrane consisting of gene products and protein complexes that are loosely bound to one of its surfaces, but not integrated into the hydrophobic region. Relationships: is a type of extrinsic component of synaptic membrane [GO:0099243]; BFO_0000050 GO:0042734 Also known as: extrinsic component of presynaptic plasma membrane Subtypes: extrinsic component of presynaptic active zone membrane [GO:0098891], extrinsic component of presynaptic endocytic zone membrane [GO:0098894] Sources: GOC:autophagy, GOC:mf